{
  "term_id": "UNKNOWN:0002",
  "term_label": "Unknown biological process",
  "gene_name": "Uncharacterized protein MISP3",
  "gene": "UniProtKB:Q96FF7",
  "gene_symbol": "MISP3"
}